{
  "gene": "UniProtKB:Q9BY19",
  "gene_symbol": "MS4A8",
  "term_id": "GO:0007166",
  "gene_name": "Membrane-spanning 4-domains subfamily A member 8",
  "term_label": "cell surface receptor signaling pathway"
}